{
  "gene": "UniProtKB:Q96L33",
  "gene_symbol": "RHOV",
  "term_id": "GO:0006897",
  "gene_name": "Rho-related GTP-binding protein RhoV",
  "term_label": "endocytosis"
}